{
  "gene_symbol": "REEP4",
  "term_id": "GO:0005881",
  "term_label": "cytoplasmic microtubule",
  "gene_name": "Receptor expression-enhancing protein 4",
  "gene": "UniProtKB:Q9H6H4"
}